{
  "term_label": "glycogen metabolic process",
  "gene_symbol": "PHKG1",
  "term_id": "GO:0005977",
  "gene_name": "Phosphorylase b kinase gamma catalytic chain, skeletal muscle_heart isoform",
  "gene": "UniProtKB:Q16816"
}